{
  "term_id": "GO:0006890",
  "gene_name": "Ras-related protein Rab-6C",
  "term_label": "retrograde vesicle-mediated transport, Golgi to endoplasmic reticulum",
  "gene": "UniProtKB:Q9H0N0",
  "gene_symbol": "RAB6C"
}